{
  "term_id": "GO:0001525",
  "term_label": "angiogenesis",
  "gene": "UniProtKB:P06756",
  "gene_name": "Integrin alpha-V",
  "gene_symbol": "ITGAV"
}